{
  "term_label": "Unknown cellular component",
  "term_id": "UNKNOWN:0003",
  "gene_name": "Zinc finger BED domain-containing protein 2",
  "gene_symbol": "ZBED2",
  "gene": "UniProtKB:Q9BTP6"
}